{
  "term_label": "DNA-(apurinic or apyrimidinic site) endonuclease activity",
  "gene": "UniProtKB:Q9UBZ4",
  "gene_name": "DNA-(apurinic or apyrimidinic site) endonuclease 2",
  "term_id": "GO:0003906",
  "gene_symbol": "APEX2"
}